{
  "term_id": "GO:0045944",
  "gene_name": "Rhombotin-2",
  "gene_symbol": "LMO2",
  "gene": "UniProtKB:P25791",
  "term_label": "positive regulation of transcription by RNA polymerase II"
}